{
  "term_label": "chromatin remodeling",
  "term_id": "GO:0006338",
  "gene": "UniProtKB:Q92830",
  "gene_symbol": "KAT2A",
  "gene_name": "Histone acetyltransferase KAT2A"
}